regulation of muscle cell differentiation [GO:0051147] (biological process) Relationships: is a type of GO:0045595; regulates muscle cell differentiation [GO:0042692] Sources: CL:0000187, GOC:ai Subtypes: negative regulation of muscle cell differentiation [GO:0051148], GO:0051149, regulation of smooth muscle cell differentiation [GO:0051150], regulation of striated muscle cell differentiation [GO:0051153] Definition: Any process that modulates the frequency, rate or extent of muscle cell differentiation.